{
  "gene_name": "Cytochrome P450 4F8",
  "term_id": "UNKNOWN:0001",
  "gene": "UniProtKB:P98187",
  "gene_symbol": "CYP4F8",
  "term_label": "Unknown molecular function"
}